{
  "gene_name": "Desumoylating isopeptidase 1",
  "term_label": "Unknown cellular component",
  "gene": "UniProtKB:Q6ICB0",
  "gene_symbol": "DESI1",
  "term_id": "UNKNOWN:0003"
}